{
  "gene_symbol": "EGF",
  "gene": "UniProtKB:P01133",
  "term_label": "plasma membrane",
  "term_id": "GO:0005886",
  "gene_name": "Pro-epidermal growth factor"
}